{
  "gene_symbol": "KIF28P",
  "term_id": "GO:0016887",
  "term_label": "ATP hydrolysis activity",
  "gene_name": "Kinesin-like protein KIF28P",
  "gene": "UniProtKB:B7ZC32"
}